{
  "term_id": "UNKNOWN:0003",
  "gene_symbol": "RLN3",
  "term_label": "Unknown cellular component",
  "gene_name": "Relaxin-3",
  "gene": "UniProtKB:Q8WXF3"
}